pancreatic PP cell development [GO:0003325] (biological process) Relationships: is a type of GO:0002064; is part of pancreatic PP cell differentiation [GO:0003312] Sources: GOC:dph Definition: The process whose specific outcome is the progression of a pancreatic PP cell over time, from its formation to the mature structure. A pancreatic polypeptide-producing cell is a cell in the pancreas that produces pancreatic polypeptide.